{
  "gene_name": "Glycerol kinase",
  "term_id": "GO:0004370",
  "gene_symbol": "GK",
  "term_label": "glycerol kinase activity",
  "gene": "UniProtKB:P32189"
}